{
  "term_label": "nucleus",
  "term_id": "GO:0005634",
  "gene": "UniProtKB:Q9NQR1",
  "gene_name": "N-lysine methyltransferase KMT5A",
  "gene_symbol": "KMT5A"
}